{
  "gene": "UniProtKB:Q14028",
  "gene_symbol": "CNGB1",
  "gene_name": "Cyclic nucleotide-gated cation channel beta-1",
  "term_label": "intracellular cyclic nucleotide activated cation channel complex",
  "term_id": "GO:0017071"
}